{
  "gene": "UniProtKB:Q8NCH0",
  "term_label": "dermatan sulfate proteoglycan metabolic process",
  "gene_symbol": "CHST14",
  "term_id": "GO:0050655",
  "gene_name": "Carbohydrate sulfotransferase 14"
}